{
  "gene_symbol": "TOMM70",
  "gene": "UniProtKB:O94826",
  "term_id": "GO:0045039",
  "gene_name": "Mitochondrial import receptor subunit TOM70",
  "term_label": "protein insertion into mitochondrial inner membrane"
}